L-alanine import across plasma membrane [GO:1904273] (biological process) References: PMID:21097500 Sources: GOC:TermGenie, GOC:kmv, GO_REF:0000075 Definition: The directed import of L-alanine from the extracellular region across the plasma membrane and into the cytosol. Relationships: is a type of amino acid import across plasma membrane [GO:0089718]; is_a GO:1904557